response to peptide hormone [GO:0043434] (biological process) Also known as: response to peptide hormone stimulus, response to polypeptide hormone stimulus Definition: Any process that results in a change in state or activity of a cell or an organism (in terms of movement, secretion, enzyme production, gene expression, etc.) as a result of a peptide hormone stimulus. A peptide hormone is any of a class of peptides that are secreted into the blood stream and have endocrine functions in living animals. Relationships: is a type of response to hormone [GO:0009725]; is_a response to nitrogen compound [GO:1901698]; is a type of response to oxygen-containing compound [GO:1901700] References: PMID:11027914, PMID:15134857 Sources: Wikipedia:Peptide_hormone Subtypes: response to insulin [GO:0032868], GO:0033762, response to luteinizing hormone [GO:0034699], response to corticotropin-releasing hormone [GO:0043435], response to growth hormone [GO:0060416], response to cholecystokinin [GO:0061847], cellular response to peptide hormone stimulus [GO:0071375], response to gonadotropin-releasing hormone [GO:0097210], response to vasopressin [GO:1904116], response to thyrotropin-releasing hormone [GO:1905225], response to prolactin [GO:1990637], response to melanocyte-stimulating hormone [GO:1990680], response to angiotensin [GO:1990776], response to endothelin [GO:1990839], response to gastrin [GO:1990867]